{
  "gene": "UniProtKB:Q8NFW9",
  "term_id": "GO:0003779",
  "gene_name": "Rab effector MyRIP",
  "term_label": "actin binding",
  "gene_symbol": "MYRIP"
}